 [go#goslim:candida] Note: Candida GO slim